positive regulation of neuron apoptotic process [GO:0043525] (biological process) Sources: GOC:go_curators, GOC:mtg_apoptosis Subtypes: positive regulation of hippocampal neuron apoptotic process [GO:0110090], GO:1903378, positive regulation of outer hair cell apoptotic process [GO:1905587], positive regulation of motor neuron apoptotic process [GO:2000673] Also known as: positive regulation of programmed cell death, neurons, up regulation of neuron apoptosis, up-regulation of neuron apoptosis, upregulation of neuron apoptosis, activation of neuron apoptosis, positive regulation of neuron apoptosis, stimulation of neuron apoptosis Definition: Any process that activates or increases the frequency, rate or extent of cell death of neurons by apoptotic process. Relationships: is a type of GO:0043065; is a type of regulation of neuron apoptotic process [GO:0043523]; positively regulates GO:0051402